Cul2-RING ubiquitin ligase complex [GO:0031462] (cellular component) Definition: A ubiquitin ligase complex in which a cullin from the Cul2 subfamily and a RING domain protein form the catalytic core; substrate specificity is conferred by an elongin-BC adaptor and a SOCS/BC box protein. References: PMID:15571813, PMID:15688063 Also known as: CBC complex, EC2S complex, ECS complex, CDL2 complex, CRL2 complex, cullin-RING ligase 2, VBC complex, SCF2 complex Relationships: is a type of cullin-RING ubiquitin ligase complex [GO:0031461]